positive regulation of epidermis development [GO:0045684] (biological process) Also known as: positive regulation of epidermal development, up regulation of epidermis development, up-regulation of epidermis development, upregulation of epidermis development, activation of epidermis development, stimulation of epidermis development, positive regulation of hypodermis development Sources: GOC:go_curators Definition: Any process that activates or increases the frequency, rate or extent of epidermis development. Subtypes: positive regulation of epidermal cell differentiation [GO:0045606] Relationships: is a type of regulation of epidermis development [GO:0045682]; is a type of GO:0051094; positively regulates GO:0008544